electron transfer activity [GO:0009055] (MF) Definition: A molecular function representing the directed movement of electrons from one molecular entity to another, typically mediated by electron carriers or acceptors, resulting in the transfer of energy and/or the reduction-oxidation (redox) transformation of chemical species. This activity is fundamental to various biological processes, including cellular respiration and photosynthesis, as well as numerous enzymatic reactions involved in metabolic pathways. Also known as: electron acceptor activity, electron donor activity, electron carrier, electron transporter activity Sources: Wikipedia:Electron_transfer Relationships: is a type of molecular_function [GO:0003674] Subtypes: cytochrome-c oxidase activity [GO:0004129], GO:0004174, GO:0008121, NADH dehydrogenase (ubiquinone) activity [GO:0008137], cytochrome bo3 ubiquinol oxidase activity [GO:0009486], plastoquinol--plastocyanin reductase activity [GO:0009496]